{
  "gene": "UniProtKB:P11150",
  "term_id": "GO:0004465",
  "term_label": "lipoprotein lipase activity",
  "gene_name": "Hepatic triacylglycerol lipase",
  "gene_symbol": "LIPC"
}